nucleic acid transmembrane transporter activity [GO:0051032] (molecular function) Subtypes: RNA transmembrane transporter activity [GO:0051033], GO:0051035 Relationships: is a type of nucleobase-containing compound transmembrane transporter activity [GO:0015932]; is_a macromolecule transmembrane transporter activity [GO:0022884]; is part of GO:0050657 Sources: GOC:ai Definition: Enables the transfer of nucleic acids from one side of a membrane to the other. Nucleic acids are single or double-stranded polynucleotides involved in the storage, transmission and transfer of genetic information.